{
  "gene_symbol": "KMT5C",
  "term_id": "GO:0042799",
  "gene": "UniProtKB:Q86Y97",
  "gene_name": "Histone-lysine N-methyltransferase KMT5C",
  "term_label": "histone H4K20 methyltransferase activity"
}